{
  "term_label": "Unknown cellular component",
  "gene_symbol": "LZIC",
  "term_id": "UNKNOWN:0003",
  "gene": "UniProtKB:Q8WZA0",
  "gene_name": "Protein LZIC"
}